{
  "gene_symbol": "LOC107984156",
  "gene": "UniProtKB:A0A0G2JMH3",
  "term_id": "GO:0005737",
  "term_label": "cytoplasm",
  "gene_name": "ADP-ribosylation factor-like protein 17 C-terminal domain-containing protein"
}